{
  "gene_symbol": "ADAM10",
  "gene": "UniProtKB:O14672",
  "term_id": "GO:0005886",
  "term_label": "plasma membrane",
  "gene_name": "Disintegrin and metalloproteinase domain-containing protein 10"
}